glycerol biosynthetic process from pyruvate [GO:0046327] (biological process) Definition: The chemical reactions and pathways resulting in the formation of glycerol, 1,2,3-propanetriol, from other compounds, including pyruvate. Sources: GOC:ai Also known as: glycerol anabolism from pyruvate, glycerol formation from pyruvate, glycerol synthesis from pyruvate, glyceroneogenesis Relationships: is a type of pyruvate metabolic process [GO:0006090]; is a type of glycerol biosynthetic process [GO:0006114]; is part of GO:0019432